translation initiation factor activity [GO:0003743] (molecular function) Sources: ISBN:0198506732 Subtypes: cap-dependent translation initiation factor activity [GO:0160296], IRES-mediated translation initiation factor activity [GO:0160297] Relationships: is a type of translation factor activity [GO:0180051]; is part of GO:0006413 Definition: Functions in the initiation of ribosome-mediated translation of mRNA into a polypeptide.